{
  "term_id": "GO:0008236",
  "term_label": "serine-type peptidase activity",
  "gene_name": "Transmembrane protease serine 3",
  "gene_symbol": "TMPRSS3",
  "gene": "UniProtKB:P57727"
}